{
  "gene": "UniProtKB:Q8N7F7",
  "term_label": "Unknown cellular component",
  "gene_symbol": "UBL4B",
  "gene_name": "Ubiquitin-like protein 4B",
  "term_id": "UNKNOWN:0003"
}